{
  "term_label": "molecular adaptor activity",
  "gene": "UniProtKB:Q9P1A6",
  "gene_name": "Disks large-associated protein 2",
  "term_id": "GO:0060090",
  "gene_symbol": "DLGAP2"
}